methionyl-initiator methionine tRNA binding [GO:1990856] (molecular function) Definition: Binding to methionine-initiator methionine tRNA. Sources: GOC:hjd, ISBN:9781555810733 Note: An example of this is eukaryotic initiation factor 2 complex, which binds the methionyl-initiator methionine tRNA during ternary complex formation. The non-acylated tRNA is not bound. Relationships: is a type of tRNA binding [GO:0000049]